CCR8 chemokine receptor binding [GO:0031733] (molecular function) Relationships: is a type of CCR chemokine receptor binding [GO:0048020] Sources: GOC:mah, GOC:nln Also known as: CCR8 chemokine receptor ligand Definition: Binding to a CCR8 chemokine receptor.